{
  "gene_name": "Selenoprotein N",
  "term_label": "calcium ion homeostasis",
  "term_id": "GO:0055074",
  "gene_symbol": "SELENON",
  "gene": "UniProtKB:Q9NZV5"
}